{
  "term_label": "wybutosine biosynthetic process",
  "term_id": "GO:0031591",
  "gene_name": "S-adenosyl-L-methionine-dependent tRNA 4-demethylwyosine synthase TYW1",
  "gene": "UniProtKB:Q9NV66",
  "gene_symbol": "TYW1"
}